{
  "gene": "UniProtKB:Q96JK9",
  "gene_symbol": "MAML3",
  "gene_name": "Mastermind-like protein 3",
  "term_id": "GO:0007221",
  "term_label": "positive regulation of transcription of Notch receptor target"
}